{
  "gene_name": "Glutamate-rich protein 5",
  "term_id": "UNKNOWN:0003",
  "term_label": "Unknown cellular component",
  "gene": "UniProtKB:Q6P6B1",
  "gene_symbol": "ERICH5"
}